tongue muscle cell differentiation [GO:0035981] (biological process) References: PMID:3393851 Sources: CL:0002673, GOC:yaf Relationships: is a type of skeletal muscle fiber differentiation [GO:0098528] Regulation: regulated by GO:2001035; negatively regulated by negative regulation of tongue muscle cell differentiation [GO:2001036]; positively regulated by positive regulation of tongue muscle cell differentiation [GO:2001037] Definition: The process in which a relatively unspecialized cell acquires specialized features of a tongue muscle cell.